sucrose metabolic process [GO:0005985] (BP) Definition: The chemical reactions and pathways involving sucrose, the disaccharide fructofuranosyl-glucopyranoside. Sources: GOC:go_curators Also known as: sucrose metabolism Subtypes: sucrose biosynthetic process [GO:0005986], sucrose catabolic process [GO:0005987] Relationships: is a type of GO:0005984